{
  "term_id": "GO:0042054",
  "term_label": "histone methyltransferase activity",
  "gene": "UniProtKB:Q99873",
  "gene_symbol": "PRMT1",
  "gene_name": "Protein arginine N-methyltransferase 1"
}